salivary nucleus development [GO:0021751] (biological process) Relationships: is_a neural nucleus development [GO:0048857]; is part of pons development [GO:0021548] Subtypes: inferior salivary nucleus development [GO:0021752], GO:0021753 Definition: The process whose specific outcome is the progression of a salivary nucleus over time, from its formation to the mature structure. Sources: GOC:cls, GOC:curators, GOC:dgh, GOC:dph, GOC:jid